{
  "term_label": "Unknown biological process",
  "gene_symbol": "SIK1B",
  "gene": "UniProtKB:A0A0B4J2F2",
  "gene_name": "Putative serine_threonine-protein kinase SIK1B",
  "term_id": "UNKNOWN:0002"
}